osmosensory signaling pathway via Sho1 osmosensor [GO:0007232] (biological process) Definition: The series of molecular signals generated in response to osmotic change, as mediated through a Sho1 osmosensor system. Also known as: osmosensory signalling pathway via Sho1 osmosensor, signal transduction during osmotic stress via Sho1 osmosensor Relationships: is a type of osmosensory signaling pathway [GO:0007231] References: PMID:26787842 Sources: GOC:jl